gamma-terpinene synthase activity [GO:0102903] (molecular function) Definition: Catalysis of the reaction: geranyl diphosphate = gamma-terpinene + diphosphoric acid. Sources: GOC:pz, RHEA:32559 Relationships: is a type of carbon-oxygen lyase activity, acting on phosphates [GO:0016838]